{
  "gene": "UniProtKB:B8ZZ34",
  "gene_name": "Protein shisa-8",
  "gene_symbol": "SHISA8",
  "term_label": "postsynaptic density",
  "term_id": "GO:0014069"
}